{
  "gene": "UniProtKB:Q9Y3E7",
  "term_label": "late endosome to vacuole transport",
  "gene_symbol": "CHMP3",
  "term_id": "GO:0045324",
  "gene_name": "Charged multivesicular body protein 3"
}